{
  "gene": "UniProtKB:P41229",
  "gene_name": "Lysine-specific demethylase 5C",
  "gene_symbol": "KDM5C",
  "term_label": "nucleus",
  "term_id": "GO:0005634"
}